regulation of SMAD protein signal transduction [GO:0060390] (biological process) Sources: GOC:BHF, GOC:dph, GOC:tb Definition: Any process that modulates the rate, frequency or extent of SMAD protein signal transduction. Subtypes: positive regulation of SMAD protein signal transduction [GO:0060391], GO:0060392 Also known as: SMAD protein import into nucleus, regulation of SMAD protein nuclear translocation Relationships: is a type of regulation of intracellular signal transduction [GO:1902531]; regulates SMAD protein signal transduction [GO:0060395]